{
  "term_id": "GO:0046839",
  "gene_symbol": "PLPP1",
  "gene": "UniProtKB:O14494",
  "term_label": "phospholipid dephosphorylation",
  "gene_name": "Phospholipid phosphatase 1"
}